positive regulation of myosin II filament organization [GO:1904901] (biological process) Relationships: is a type of GO:0043519; is a type of positive regulation of cytoskeleton organization [GO:0051495]; is a type of positive regulation of supramolecular fiber organization [GO:1902905]; positively regulates myosin II filament organization [GO:0031038] Also known as: positive regulation of myosin II filament organisation, up regulation of myosin II filament organisation, up regulation of myosin II filament organization, up-regulation of myosin II filament organisation, up-regulation of myosin II filament organization, upregulation of myosin II filament organisation, upregulation of myosin II filament organization, activation of myosin II filament organisation, activation of myosin II filament organization, activation of myosin II filament assembly or disassembly, activation of myosin II polymerization or depolymerization, positive regulation of myosin II filament assembly or disassembly, positive regulation of myosin II polymerization or depolymerization, up regulation of myosin II filament assembly or disassembly, up regulation of myosin II polymerization or depolymerization, up-regulation of myosin II filament assembly or disassembly, up-regulation of myosin II polymerization or depolymerization, upregulation of myosin II filament assembly or disassembly, upregulation of myosin II polymerization or depolymerization Subtypes: GO:1905511 References: PMID:22761445 Sources: GOC:TermGenie, GO_REF:0000058 Definition: Any process that activates or increases the frequency, rate or extent of myosin II filament organization.